cell-cell recognition [GO:0009988] (biological process) Relationships: is a type of cell recognition [GO:0008037] Subtypes: immunological synapse formation [GO:0001771], sperm-egg recognition [GO:0035036], male-female gamete recognition during double fertilization forming a zygote and endosperm [GO:0080173], cell-cell self recognition [GO:0097656] Sources: ISBN:0824072820 Definition: Cell recognition between cells. May involve the formation of specialized cell junctions.